{
  "gene_symbol": "LINC02913",
  "term_id": "UNKNOWN:0003",
  "term_label": "Unknown cellular component",
  "gene": "UniProtKB:Q8NAJ2",
  "gene_name": "Putative uncharacterized protein encoded by LINC02913"
}